maintenance of cell polarity [GO:0030011] (biological process) Definition: The maintenance of established anisotropic intracellular organization or cell growth patterns. Sources: GOC:mah Relationships: is a type of establishment or maintenance of cell polarity [GO:0007163] Subtypes: maintenance of apical/basal cell polarity [GO:0035090], maintenance of neuroblast polarity [GO:0045201]